response to absence of light [GO:0009646] (biological process) Also known as: response to darkness Relationships: is a type of response to light intensity [GO:0009642] Sources: GOC:go_curators Definition: Any process that results in a change in state or activity of a cell or an organism (in terms of movement, secretion, enzyme production, gene expression, etc.) as a result of an absence of light stimuli. Subtypes: GO:0009647, cellular response to absence of light [GO:0071485]